{
  "gene_name": "Metal transporter CNNM3",
  "term_label": "plasma membrane",
  "term_id": "GO:0005886",
  "gene": "UniProtKB:Q8NE01",
  "gene_symbol": "CNNM3"
}